nucleoside ribosyltransferase activity [GO:0050147] (MF) Sources: EC:2.4.2.5, MetaCyc:NUCLEOSIDE-RIBOSYLTRANSFERASE-RXN Definition: Catalysis of the reaction: D-ribosyl-base1 + base2 = D-ribosyl-base2 + base1. Relationships: is a type of GO:0016763 Also known as: nucleoside N-ribosyltransferase activity, nucleoside:purine(pyrimidine) D-ribosyltransferase activity